{
  "gene_name": "Lymphotoxin-alpha",
  "term_label": "cell surface receptor signaling pathway",
  "term_id": "GO:0007166",
  "gene": "UniProtKB:P01374",
  "gene_symbol": "LTA"
}